{
  "term_id": "GO:0008289",
  "gene_symbol": "DEFB107A",
  "term_label": "lipid binding",
  "gene_name": "Beta-defensin 107",
  "gene": "UniProtKB:Q8IZN7"
}